{
  "gene_name": "2'-5'-oligoadenylate synthase 2",
  "term_id": "GO:0140374",
  "term_label": "antiviral innate immune response",
  "gene_symbol": "OAS2",
  "gene": "UniProtKB:P29728"
}